{
  "term_label": "Unknown cellular component",
  "gene_symbol": "ZNF800",
  "gene": "UniProtKB:Q2TB10",
  "gene_name": "Zinc finger protein 800",
  "term_id": "UNKNOWN:0003"
}